negative regulation of N-terminal protein palmitoylation [GO:0060262] (biological process) Relationships: is a type of regulation of N-terminal protein palmitoylation [GO:0060254]; is a type of negative regulation of protein lipidation [GO:1903060]; negatively regulates N-terminal protein palmitoylation [GO:0006500] Sources: GOC:dph, GOC:tb Definition: Any process that decreases the rate frequency or extent of the covalent attachment of a palmitoyl group to the N-terminal amino acid residue of a protein.